{
  "gene": "UniProtKB:Q8NHQ1",
  "gene_name": "Centrosomal protein of 70 kDa",
  "gene_symbol": "CEP70",
  "term_id": "UNKNOWN:0001",
  "term_label": "Unknown molecular function"
}